{
  "gene_symbol": "NRP1",
  "term_id": "GO:0030947",
  "gene_name": "Neuropilin-1",
  "gene": "UniProtKB:O14786",
  "term_label": "regulation of vascular endothelial growth factor receptor signaling pathway"
}